{
  "gene": "UniProtKB:Q9BXS6",
  "gene_symbol": "NUSAP1",
  "term_label": "establishment of mitotic spindle localization",
  "gene_name": "Nucleolar and spindle-associated protein 1",
  "term_id": "GO:0040001"
}